{
  "gene_name": "Olfactory receptor 1B1",
  "gene": "UniProtKB:Q8NGR6",
  "term_id": "GO:0005886",
  "term_label": "plasma membrane",
  "gene_symbol": "OR1B1"
}